prothylakoid [GO:0042649] (cellular component) Definition: Underdeveloped thylakoids found in etioplasts, lacking competent photosynthetic membranes. Rapidly develop into mature thylakoids in the presence of light. References: PMID:11532175 Sources: GOC:jl Relationships: is a type of plastid thylakoid [GO:0031976]; is part of etioplast [GO:0009513]